{
  "term_label": "DNA-binding transcription factor activity, RNA polymerase II-specific",
  "gene_symbol": "SATB1",
  "gene_name": "DNA-binding protein SATB1",
  "gene": "UniProtKB:Q01826",
  "term_id": "GO:0000981"
}